{
  "gene_name": "Brain-derived neurotrophic factor",
  "term_id": "GO:0043524",
  "term_label": "negative regulation of neuron apoptotic process",
  "gene_symbol": "BDNF",
  "gene": "UniProtKB:P23560"
}